{
  "gene_symbol": "ATP5F1B",
  "term_id": "GO:0046933",
  "gene_name": "ATP synthase subunit beta, mitochondrial",
  "gene": "UniProtKB:P06576",
  "term_label": "proton-transporting ATP synthase activity, rotational mechanism"
}